{
  "gene": "UniProtKB:Q13087",
  "gene_name": "Protein disulfide-isomerase A2",
  "term_id": "GO:0006457",
  "term_label": "protein folding",
  "gene_symbol": "PDIA2"
}